{
  "gene_symbol": "MRE11",
  "gene": "UniProtKB:P49959",
  "term_id": "GO:0000014",
  "gene_name": "Double-strand break repair protein MRE11",
  "term_label": "single-stranded DNA endodeoxyribonuclease activity"
}